transcriptional start site selection at RNA polymerase III promoter [GO:0001175] (biological process) Definition: Any process involved in the selection of the specific location within the template strand of an RNA polymerase III promoter for hybridization of the cognate ribonucleotides and formation of first phosphodiester bond within the nascent transcript. Sources: GOC:txnOH Relationships: is a type of GO:0001173; is part of GO:0006384